{
  "term_id": "GO:0006357",
  "gene_symbol": "DMTF1",
  "gene": "UniProtKB:Q9Y222",
  "gene_name": "Cyclin-D-binding Myb-like transcription factor 1",
  "term_label": "regulation of transcription by RNA polymerase II"
}